{
  "gene_name": "A disintegrin and metalloproteinase with thrombospondin motifs 9",
  "gene_symbol": "ADAMTS9",
  "term_label": "extracellular matrix organization",
  "gene": "UniProtKB:Q9P2N4",
  "term_id": "GO:0030198"
}